4-methylumbelliferyl-beta-D-glucopyranoside beta-glucosidase activity [GO:0080081] (molecular function) Definition: Catalysis of the hydrolysis of glucosidic link in 4-methylumbelliferyl-beta-D-glucopyranoside. References: PMID:15604686 Relationships: is a type of beta-glucosidase activity [GO:0008422]